{
  "term_label": "dendrite",
  "term_id": "GO:0030425",
  "gene": "UniProtKB:Q9UL51",
  "gene_symbol": "HCN2",
  "gene_name": "Potassium_sodium hyperpolarization-activated cyclic nucleotide-gated channel 2"
}